{
  "term_label": "nucleus",
  "gene_name": "Radiation-inducible immediate-early gene IEX-1",
  "term_id": "GO:0005634",
  "gene_symbol": "IER3",
  "gene": "UniProtKB:P46695"
}